{
  "term_id": "GO:0005925",
  "gene": "UniProtKB:Q8WUP2",
  "gene_name": "Filamin-binding LIM protein 1",
  "term_label": "focal adhesion",
  "gene_symbol": "FBLIM1"
}